{
  "gene_name": "Myosin light chain kinase 2, skeletal_cardiac muscle",
  "term_label": "cytoplasm",
  "term_id": "GO:0005737",
  "gene": "UniProtKB:Q9H1R3",
  "gene_symbol": "MYLK2"
}